protein domain specific binding [GO:0019904] (molecular function) Definition: Binding to a specific domain of a protein. Relationships: is a type of protein binding [GO:0005515] Also known as: protein domain-specific binding Sources: GOC:go_curators Subtypes: FH1 domain binding [GO:0017058], SH3 domain binding [GO:0017124], GO:0030165, LIM domain binding [GO:0030274], GO:0030275, TPR domain binding [GO:0030911], POZ domain binding [GO:0031208], NACHT domain binding [GO:0032089], Pyrin domain binding [GO:0032090], GO:0032093, GO:0032399, GBD domain binding [GO:0032427], FFAT motif binding [GO:0033149], GO:0035500, MH1 domain binding [GO:0035501], GO:0035851, death effector domain binding [GO:0035877], GAF domain binding [GO:0036004], GO:0036143, GO:0042169, PH domain binding [GO:0042731], HLH domain binding [GO:0043398], Rel homology domain binding [GO:0044197], zf-TRAF domain binding [GO:0044198], AF-2 domain binding [GO:0050682], AF-1 domain binding [GO:0050683], DNA binding domain binding [GO:0050692], LBD domain binding [GO:0050693], GO:0050699, CARD domain binding [GO:0050700], RS domain binding [GO:0050733], BH domain binding [GO:0051400], GO:0051401, PTB domain binding [GO:0051425], GO:0055131, EGF repeat binding [GO:0061788], armadillo repeat domain binding [GO:0070016], titin Z domain binding [GO:0070080], chromo shadow domain binding [GO:0070087], GO:0070513, C2H2 zinc finger domain binding [GO:0070742], POU domain binding [GO:0070974], FHA domain binding [GO:0070975], TIR domain binding [GO:0070976], SET domain binding [GO:0070984], ankyrin repeat binding [GO:0071532], RING-like zinc finger domain binding [GO:0071535], RIP homotypic interaction motif binding [GO:0071551], CAP-Gly domain binding [GO:0071794], HMG box domain binding [GO:0071837], CRD domain binding [GO:0071906], WD40-repeat domain binding [GO:0071987], GO:0090488, GO:0090541, ELYC domain binding [GO:0090542], MATH domain binding [GO:0090736], L27 domain binding [GO:0097016], DH domain binding [GO:0097161], GO:0097162, disordered domain specific binding [GO:0097718], LEM domain binding [GO:0097726], GO:0098750, FMN-binding domain binding [GO:0101016], C2 domain binding [GO:0110036], EH domain binding [GO:1990175], type-I dockerin domain binding [GO:1990308], type-II dockerin domain binding [GO:1990309], type-III dockerin domain binding [GO:1990310], GO:1990311, GO:1990312, type-III cohesin domain binding [GO:1990313], F-box domain binding [GO:1990444], GO:1990525, F-bar domain binding [GO:1990808]